protein kinase 5 complex [GO:0016533] (cellular component) Relationships: is a type of serine/threonine protein kinase complex [GO:1902554] Also known as: cyclin-dependent protein kinase 5 holoenzyme complex References: PMID:15689152 Definition: A protein complex that has protein serine/threonine kinase activity; in mammals composed of catalytic subunit CDK5 and regulatory subunits CDK5R1 or CDK5R2. Contrary to its gene symbol, CDK5 is not cyclin-dependent.